{
  "gene_name": "Ras-related protein Rab-1B",
  "gene_symbol": "RAB1B",
  "gene": "UniProtKB:Q9H0U4",
  "term_label": "endomembrane system",
  "term_id": "GO:0012505"
}